{
  "term_id": "GO:0051966",
  "gene": "UniProtKB:Q14833",
  "gene_symbol": "GRM4",
  "term_label": "regulation of synaptic transmission, glutamatergic",
  "gene_name": "Metabotropic glutamate receptor 4"
}